{
  "gene_name": "Serine_threonine-protein kinase Nek10",
  "term_label": "protein kinase complex",
  "term_id": "GO:1902911",
  "gene_symbol": "NEK10",
  "gene": "UniProtKB:Q6ZWH5"
}